{
  "gene_symbol": "ABCD4",
  "gene": "UniProtKB:O14678",
  "term_id": "GO:0006635",
  "gene_name": "Lysosomal cobalamin transporter ABCD4",
  "term_label": "fatty acid beta-oxidation"
}